{
  "gene": "UniProtKB:Q9GZZ6",
  "gene_symbol": "CHRNA10",
  "term_label": "regulation of membrane potential",
  "gene_name": "Neuronal acetylcholine receptor subunit alpha-10",
  "term_id": "GO:0042391"
}